{
  "term_label": "cytosol",
  "gene": "UniProtKB:O94806",
  "gene_name": "Serine_threonine-protein kinase D3",
  "gene_symbol": "PRKD3",
  "term_id": "GO:0005829"
}